carbohydrate localization [GO:0052575] (biological process) Also known as: carbohydrate localisation Relationships: is a type of macromolecule localization [GO:0033036] Subtypes: carbohydrate storage [GO:0052576] Definition: Any process in which a carbohydrate is transported to, or maintained in, a specific location. Carbohydrates are any of a group of organic compounds based of the general formula Cx(H2O)y. Sources: GOC:mah